{
  "gene": "UniProtKB:Q9BSW7",
  "gene_name": "Synaptotagmin-17",
  "gene_symbol": "SYT17",
  "term_id": "GO:0005544",
  "term_label": "calcium-dependent phospholipid binding"
}